{
  "gene_name": "Eukaryotic translation initiation factor 3 subunit F",
  "term_label": "translation initiation factor activity",
  "term_id": "GO:0003743",
  "gene": "UniProtKB:O00303",
  "gene_symbol": "EIF3F"
}